{
  "gene": "UniProtKB:Q6NXP2",
  "gene_name": "Golgi-associated RAB2 interactor protein 1A",
  "term_id": "UNKNOWN:0002",
  "gene_symbol": "GARIN1A",
  "term_label": "Unknown biological process"
}